AUC codon-amino acid adaptor activity [GO:0033434] (molecular function) Sources: GOC:mah Note: Note that in the standard genetic code, ATC codes for isoleucine. Definition: A triplet codon-amino acid adaptor activity that recognizes an AUC codon. Relationships: is a type of triplet codon-amino acid adaptor activity [GO:0030533] Also known as: ATC codon-amino acid adaptor activity, isoleucine tRNA